{
  "gene_name": "Mediator of RNA polymerase II transcription subunit 15",
  "gene_symbol": "MED15",
  "term_id": "GO:0070847",
  "term_label": "core mediator complex",
  "gene": "UniProtKB:Q96RN5"
}